response to isobutanol [GO:1902665] (biological process) Relationships: is a type of response to alcohol [GO:0097305] Definition: Any process that results in a change in state or activity of a cell or an organism (in terms of movement, secretion, enzyme production, gene expression, etc.) as a result of an isobutanol stimulus. References: PMID:24014527 Sources: GOC:TermGenie, GOC:mengo_curators, GO_REF:0000071 Also known as: response to 2-methylpropan-1-ol, process resulting in tolerance to isobutanol